mammary duct terminal end bud growth [GO:0060763] (biological process) Definition: The morphogenetic growth of the large, club-shaped terminal end of a mammary gland duct during prepubertal growth and during puberty. Relationships: is a type of developmental growth involved in morphogenesis [GO:0060560]; BFO_0000050 mammary gland duct morphogenesis [GO:0060603] References: PMID:10804170 Sources: GOC:dph